{
  "term_id": "GO:2001244",
  "gene": "UniProtKB:Q9Y6J8",
  "term_label": "positive regulation of intrinsic apoptotic signaling pathway",
  "gene_symbol": "STYXL1",
  "gene_name": "Serine_threonine_tyrosine-interacting-like protein 1"
}